{
  "term_id": "UNKNOWN:0003",
  "gene": "UniProtKB:Q6NSI1",
  "term_label": "Unknown cellular component",
  "gene_name": "Putative ankyrin repeat domain-containing protein 26-like protein",
  "gene_symbol": "ANKRD26P1"
}